deoxyribonucleoside triphosphate catabolic process [GO:0009204] (biological process) Definition: The chemical reactions and pathways resulting in the breakdown of a deoxyribonucleoside triphosphate, a compound consisting of a nucleobase linked to a deoxyribose sugar esterified with triphosphate on the sugar. Sources: GOC:go_curators, ISBN:0198506732 Also known as: deoxyribonucleoside triphosphate breakdown, deoxyribonucleoside triphosphate catabolism, deoxyribonucleoside triphosphate degradation Subtypes: purine deoxyribonucleoside triphosphate catabolic process [GO:0009217] Relationships: is a type of GO:0009143; is a type of deoxyribonucleoside triphosphate metabolic process [GO:0009200]